{
  "term_id": "UNKNOWN:0001",
  "gene_symbol": "PROSER3",
  "term_label": "Unknown molecular function",
  "gene": "UniProtKB:Q2NL68",
  "gene_name": "Proline and serine-rich protein 3"
}